regulation of iridophore differentiation [GO:0050937] (BP) Subtypes: GO:0050943, positive regulation of iridophore differentiation [GO:0050945] Definition: Any process that modulates the frequency, rate or extent of iridophore differentiation. Sources: GOC:ai Relationships: is a type of regulation of pigment cell differentiation [GO:0050932]; regulates iridophore differentiation [GO:0050935]